{
  "term_id": "GO:0000122",
  "gene": "UniProtKB:Q8TAX0",
  "term_label": "negative regulation of transcription by RNA polymerase II",
  "gene_symbol": "OSR1",
  "gene_name": "Protein odd-skipped-related 1"
}